{
  "gene_symbol": "ARFGAP1",
  "gene_name": "ADP-ribosylation factor GTPase-activating protein 1",
  "term_label": "regulation of ARF protein signal transduction",
  "term_id": "GO:0032012",
  "gene": "UniProtKB:Q8N6T3"
}